positive regulation of DNA recombination [GO:0045911] (BP) Sources: GOC:go_curators Subtypes: activation of recombination (HML) [GO:0007536], positive regulation of reciprocal meiotic recombination [GO:0010845], positive regulation of isotype switching [GO:0045830], GO:0045951, positive regulation of DNA recombination at centromere [GO:0061807], positive regulation of DNA recombination at telomere [GO:0072696], positive regulation of single-strand break repair via homologous recombination [GO:1903112], positive regulation of double-strand break repair via homologous recombination [GO:1905168] Also known as: up regulation of DNA recombination, up-regulation of DNA recombination, upregulation of DNA recombination, activation of DNA recombination, stimulation of DNA recombination Relationships: is a type of regulation of DNA recombination [GO:0000018]; is a type of GO:0051054; positively regulates DNA recombination [GO:0006310] Definition: Any process that activates or increases the frequency, rate or extent of DNA recombination.